mitochondria-associated ubiquitin-dependent protein catabolic process [GO:0072671] (biological process) Also known as: MAD, mitochondria-associated protein catabolic process, mitochondria-associated protein degradation, mitochondrion-associated protein catabolic process Definition: The chemical reactions and pathways resulting in the breakdown of proteins transported from mitochondria and targeted to cytoplasmic proteasomes for degradation as a response to oxidative stress conditions. References: PMID:21070972, PMID:21109188 Sources: GOC:mcc Relationships: is a type of proteasome-mediated ubiquitin-dependent protein catabolic process [GO:0043161]